{
  "gene": "UniProtKB:P78316",
  "term_id": "GO:0032040",
  "gene_symbol": "NOP14",
  "term_label": "small-subunit processome",
  "gene_name": "Nucleolar protein 14"
}